{
  "term_label": "angiogenesis",
  "gene": "UniProtKB:P08514",
  "gene_name": "Integrin alpha-IIb",
  "gene_symbol": "ITGA2B",
  "term_id": "GO:0001525"
}